4-hydroxyphenylpyruvate oxidase activity [GO:0018490] (molecular function) Also known as: 4-hydroxyphenylpyruvate:oxygen oxidoreductase (decarboxylating) Sources: RHEA:17197 Definition: Catalysis of the reaction: 2 3-(4-hydroxyphenyl)pyruvate + O2 = 2 4-hydroxyphenylacetate + 2 CO2. Relationships: is a type of oxidoreductase activity, acting on the aldehyde or oxo group of donors, oxygen as acceptor [GO:0016623]